{
  "gene_name": "F-box only protein 10",
  "term_label": "Unknown molecular function",
  "gene_symbol": "FBXO10",
  "gene": "UniProtKB:Q9UK96",
  "term_id": "UNKNOWN:0001"
}